regulation of mitochondrial fission [GO:0090140] (BP) Also known as: regulation of mitochondrial division Sources: GOC:ascb_2009, GOC:dph, GOC:tb Relationships: is a type of regulation of mitochondrion organization [GO:0010821]; is a type of regulation of anatomical structure morphogenesis [GO:0022603]; regulates mitochondrial fission [GO:0000266] Definition: Any process that modulates the rate, frequency or extent of mitochondrial fission. Mitochondrial fission is the division of a mitochondrion within a cell to form two or more separate mitochondrial compartments. Subtypes: positive regulation of mitochondrial fission [GO:0090141], negative regulation of mitochondrial fission [GO:0090258]